{
  "gene": "UniProtKB:Q8IY31",
  "gene_symbol": "IFT20",
  "term_label": "ciliary base",
  "gene_name": "Intraflagellar transport protein 20 homolog",
  "term_id": "GO:0097546"
}